aerobactin transport [GO:0019271] (biological process) Relationships: is a type of tricarboxylic acid transport [GO:0006842]; is a type of modified amino acid transport [GO:0072337] References: PMID:23192658 Sources: GOC:ai Definition: The directed movement of the hydroxamate iron transport compound aerobactin into, out of or within a cell, or between cells, by means of some agent such as a transporter or pore. Aerobactin (C22H36N4O13) is a conjugate of 6-(N-acetyl-N-hydroxylamine)-2-aminohexanoic acid and citric acid.